{
  "term_label": "Unknown biological process",
  "gene_symbol": "RIG",
  "gene": "UniProtKB:Q13278",
  "term_id": "UNKNOWN:0002",
  "gene_name": "Putative protein RIG"
}